{
  "gene": "UniProtKB:Q9UM07",
  "gene_name": "Protein-arginine deiminase type-4",
  "gene_symbol": "PADI4",
  "term_label": "histone arginine deiminase activity",
  "term_id": "GO:0140794"
}